{
  "gene": "UniProtKB:Q9HAV4",
  "gene_name": "Exportin-5",
  "term_label": "RNA export from nucleus",
  "gene_symbol": "XPO5",
  "term_id": "GO:0006405"
}